{
  "gene_name": "Reticulon-3",
  "term_id": "UNKNOWN:0001",
  "gene_symbol": "RTN3",
  "term_label": "Unknown molecular function",
  "gene": "UniProtKB:O95197"
}